{
  "gene_name": "Homeobox protein Hox-D10",
  "term_id": "GO:0006357",
  "term_label": "regulation of transcription by RNA polymerase II",
  "gene": "UniProtKB:P28358",
  "gene_symbol": "HOXD10"
}